{
  "gene_name": "Fibrillin-2",
  "gene_symbol": "FBN2",
  "gene": "UniProtKB:P35556",
  "term_label": "extracellular matrix structural constituent",
  "term_id": "GO:0005201"
}